{
  "gene_symbol": "MYL5",
  "term_id": "GO:0005737",
  "gene": "UniProtKB:Q02045",
  "term_label": "cytoplasm",
  "gene_name": "Myosin light chain 5"
}